{
  "gene_symbol": "HNRNPCL2",
  "gene_name": "Heterogeneous nuclear ribonucleoprotein C-like 2",
  "term_id": "UNKNOWN:0002",
  "gene": "UniProtKB:B2RXH8",
  "term_label": "Unknown biological process"
}